{
  "gene": "UniProtKB:O00221",
  "term_label": "cytoplasm",
  "term_id": "GO:0005737",
  "gene_symbol": "NFKBIE",
  "gene_name": "NF-kappa-B inhibitor epsilon"
}